{
  "gene_symbol": "KPLCE",
  "term_label": "Unknown biological process",
  "gene": "UniProtKB:Q5T750",
  "gene_name": "Protein KPLCE",
  "term_id": "UNKNOWN:0002"
}